{
  "gene_name": "Myb_SANT-like DNA-binding domain-containing protein 7",
  "gene_symbol": "MSANTD7",
  "term_id": "UNKNOWN:0001",
  "gene": "UniProtKB:A0A1W2PQ72",
  "term_label": "Unknown molecular function"
}